{
  "term_id": "GO:0005762",
  "term_label": "mitochondrial large ribosomal subunit",
  "gene_name": "Large ribosomal subunit protein mL54",
  "gene_symbol": "MRPL54",
  "gene": "UniProtKB:Q6P161"
}